tripeptide transmembrane transport [GO:0035443] (biological process) Definition: The directed movement of a tripeptide across a membrane by means of some agent such as a transporter or pore. A tripeptide is a compound containing three amino acids linked together by peptide bonds. Sources: GOC:vw Also known as: tripeptide membrane transport Note: Note that this term is not intended for use in annotating lateral movement within membranes. Relationships: is a type of GO:0035672; is a type of tripeptide transport [GO:0042939] Subtypes: GO:0034775, GO:0140207